{
  "gene_symbol": "IGHD3-10",
  "gene_name": "Immunoglobulin heavy diversity 3-10 (Fragment)",
  "term_id": "UNKNOWN:0001",
  "term_label": "Unknown molecular function",
  "gene": "UniProtKB:A0A0J9YXN1"
}